{
  "term_id": "GO:0000055",
  "term_label": "ribosomal large subunit export from nucleus",
  "gene": "UniProtKB:Q9NVU7",
  "gene_symbol": "SDAD1",
  "gene_name": "Protein SDA1 homolog"
}